{
  "gene_symbol": "CUL1",
  "term_id": "GO:0005634",
  "gene_name": "Cullin-1",
  "term_label": "nucleus",
  "gene": "UniProtKB:Q13616"
}